{
  "term_id": "UNKNOWN:0003",
  "gene": "UniProtKB:Q8N859",
  "gene_symbol": "ZNF713",
  "gene_name": "Zinc finger protein 713",
  "term_label": "Unknown cellular component"
}